{
  "gene_name": "ER membrane protein complex subunit 1",
  "term_label": "EMC complex",
  "term_id": "GO:0072546",
  "gene_symbol": "EMC1",
  "gene": "UniProtKB:Q8N766"
}